negative regulation of metaphase/anaphase transition of meiosis I [GO:1905187] (biological process) Definition: Any process that stops, prevents or reduces the frequency, rate or extent of metaphase/anaphase transition of meiosis I. References: PMID:21389117 Sources: GOC:TermGenie, GO_REF:0000058 Relationships: is a type of negative regulation of metaphase/anaphase transition of meiotic cell cycle [GO:1902103]; is a type of GO:1905186; RO_0002212 GO:1990949